CoB--CoM heterodisulfide reductase activity [GO:0051912] (molecular function) Definition: Catalysis of the reaction: coenzyme B + coenzyme M + methanophenazine = N-{7-[(2-sulfoethyl)dithio]heptanoyl}-3-O-phospho-L-threonine + dihydromethanophenazine. Relationships: is a type of oxidoreductase activity, acting on a sulfur group of donors [GO:0016667] Sources: RHEA:18085 Also known as: heterodisulfide reductase activity, CoB-CoM heterodisulfide reductase activity, coenzyme B--coenzyme M heterodisulfide reductase activity, coenzyme B:coenzyme M:methanophenazine oxidoreductase activity, coenzyme-M-7-mercaptoheptanoylthreonine-phosphate-heterodisulfide hydrogenase activity, soluble heterodisulfide reductase activity